{
  "term_label": "Unknown cellular component",
  "gene_symbol": "FAM107B",
  "term_id": "UNKNOWN:0003",
  "gene_name": "Protein FAM107B",
  "gene": "UniProtKB:Q9H098"
}